centriole assembly [GO:0098534] (biological process) Relationships: is a type of microtubule organizing center organization [GO:0031023]; is a type of membraneless organelle assembly [GO:0140694] References: PMID:24075808 Sources: GOC:dos Definition: A cellular process that results in the assembly of one or more centrioles. Subtypes: centriole replication [GO:0007099], GO:0097742